{
  "gene_symbol": "PARK7",
  "term_id": "GO:0016684",
  "term_label": "oxidoreductase activity, acting on peroxide as acceptor",
  "gene": "UniProtKB:Q99497",
  "gene_name": "Parkinson disease protein 7"
}